{
  "gene_symbol": "TOR1B",
  "gene": "UniProtKB:O14657",
  "term_label": "endoplasmic reticulum lumen",
  "gene_name": "Torsin-1B",
  "term_id": "GO:0005788"
}